{
  "term_id": "UNKNOWN:0001",
  "gene_symbol": "C21orf62",
  "gene": "UniProtKB:Q9NYP8",
  "gene_name": "Uncharacterized protein C21orf62",
  "term_label": "Unknown molecular function"
}